{
  "gene": "UniProtKB:A0PJX2",
  "term_label": "response to oxidative stress",
  "gene_name": "TLD domain-containing protein 2",
  "gene_symbol": "TLDC2",
  "term_id": "GO:0006979"
}